{
  "gene": "UniProtKB:A8MW99",
  "gene_symbol": "MEI4",
  "gene_name": "Meiosis-specific protein MEI4",
  "term_label": "meiotic DNA double-strand break formation",
  "term_id": "GO:0042138"
}